negative regulation of torso signaling pathway [GO:0120177] (biological process) Definition: Any process that stops, prevents, or reduces the frequency, rate or extent of the torso signaling pathway. References: PMID:23732470 Sources: GOC:ha Relationships: is a type of GO:0009968; is a type of GO:0120175; negatively regulates GO:0008293